{
  "term_id": "GO:0042796",
  "gene": "UniProtKB:Q92966",
  "gene_name": "snRNA-activating protein complex subunit 3",
  "gene_symbol": "SNAPC3",
  "term_label": "snRNA transcription by RNA polymerase III"
}